{
  "gene_symbol": "CPLX3",
  "term_id": "GO:0043195",
  "gene": "UniProtKB:Q8WVH0",
  "term_label": "terminal bouton",
  "gene_name": "Complexin-3"
}